neuromast hair cell differentiation involved in neuromast regeneration [GO:0070658] (biological process) Definition: Differentiation of new neuromast sensory hair cells to replace those lost or destroyed by injury. References: PMID:19381250 Sources: GOC:dsf Relationships: is a type of neuromast hair cell differentiation [GO:0048886]; is a type of mechanoreceptor differentiation involved in mechanosensory epithelium regeneration [GO:0070656]; is part of GO:0070657